pyridine nucleoside biosynthetic process [GO:0071589] (biological process) Subtypes: nicotinamide riboside biosynthetic process [GO:0071590], GO:0071592 Also known as: pyridine nucleoside anabolism, pyridine nucleoside biosynthesis, pyridine nucleoside formation, pyridine nucleoside synthesis Definition: The chemical reactions and pathways resulting in the formation of any pyridine nucleoside, one of a family of organic molecules consisting of a pyridine base covalently bonded to a sugar, usually ribose. Sources: GOC:mah Relationships: is a type of nucleoside biosynthetic process [GO:0009163]; is a type of pyridine nucleoside metabolic process [GO:0070637]; is a type of pyridine-containing compound biosynthetic process [GO:0072525]